{
  "gene_name": "Hyaluronan and proteoglycan link protein 3",
  "term_id": "GO:0007417",
  "gene": "UniProtKB:Q96S86",
  "gene_symbol": "HAPLN3",
  "term_label": "central nervous system development"
}